{
  "gene_name": "Peripheral plasma membrane protein CASK",
  "term_label": "regulation of neurotransmitter secretion",
  "gene": "UniProtKB:O14936",
  "gene_symbol": "CASK",
  "term_id": "GO:0046928"
}